{
  "term_label": "protein kinase binding",
  "gene": "UniProtKB:Q86Y37",
  "gene_symbol": "CACUL1",
  "gene_name": "CDK2-associated and cullin domain-containing protein 1",
  "term_id": "GO:0019901"
}